{
  "gene_name": "Large ribosomal subunit protein eL24",
  "term_label": "mRNA binding",
  "gene_symbol": "RPL24",
  "term_id": "GO:0003729",
  "gene": "UniProtKB:P83731"
}